pyridoxal 5'-phosphate synthase (glutamine hydrolysing) activity [GO:0036381] (molecular function) Definition: Catalysis of the reaction: D-ribose 5-phosphate + D-glyceraldehyde 3-phosphate + L-glutamine = pyridoxal 5'-phosphate + L-glutamate + 3 H2O + phosphate. The reaction occurs in two steps: L-glutamine + H2O = L-glutamate + NH3, and subsequently D-ribose 5-phosphate + D-glyceraldehyde 3-phosphate + NH3 = pyridoxal 5'-phosphate + 4 H2O + phosphate. Sources: EC:4.3.3.6, GOC:rs Also known as: PdxST activity, pyridoxal 5'-phosphate synthase (glutamine hydrolyzing) activity Relationships: is_a GO:0016843